{
  "term_id": "GO:0005737",
  "term_label": "cytoplasm",
  "gene": "UniProtKB:O43255",
  "gene_name": "E3 ubiquitin-protein ligase SIAH2",
  "gene_symbol": "SIAH2"
}